{
  "gene": "UniProtKB:Q9BQE4",
  "gene_symbol": "SELENOS",
  "term_id": "GO:0036513",
  "term_label": "Derlin-1 retrotranslocation complex",
  "gene_name": "Selenoprotein S"
}